regulation of respiratory burst [GO:0060263] (biological process) Definition: Any process that modulates the rate frequency or extent of a phase of elevated metabolic activity, during which oxygen consumption increases; this leads to the production, by an NADH dependent system, of hydrogen peroxide (H2O2), superoxide anions and hydroxyl radicals. Sources: GOC:dph, GOC:tb Relationships: is a type of GO:0019222; regulates respiratory burst [GO:0045730] Subtypes: regulation of respiratory burst involved in inflammatory response [GO:0060264], positive regulation of respiratory burst [GO:0060267], GO:0060268